glycogen biosynthetic process via UDP-glucose [GO:0160249] (biological process) Sources: MetaCyc:PWY-5067 Relationships: is_a GO:0005978 Definition: The chemical reactions and pathways resulting in the formation of glycogen, a polydisperse, highly branched glucan composed of chains of D-glucose residues, occurring through a UDP-glucose intermediate.